{
  "gene_name": "Probable transmembrane reductase CYB561D1",
  "term_label": "Unknown biological process",
  "term_id": "UNKNOWN:0002",
  "gene_symbol": "CYB561D1",
  "gene": "UniProtKB:Q8N8Q1"
}